{
  "term_id": "GO:0015630",
  "gene_name": "Septin-5",
  "gene": "UniProtKB:Q99719",
  "term_label": "microtubule cytoskeleton",
  "gene_symbol": "SEPTIN5"
}